{
  "gene_symbol": "ABHD1",
  "term_id": "GO:0051792",
  "term_label": "medium-chain fatty acid biosynthetic process",
  "gene_name": "Protein ABHD1",
  "gene": "UniProtKB:Q96SE0"
}